homogalacturonan biosynthetic process [GO:0010289] (biological process) Relationships: is a type of GO:0010394; is a type of cell wall pectin biosynthetic process [GO:0052325] Definition: The chemical reactions and pathways resulting in the formation of the pectidic homogalacturonan, characterized by a backbone of (1->4)-linked alpha-D-GalpA residues that can be methyl-esterified at C-6 and carry acetyl groups on O-2 and O-3. References: PMID:12913136, PMID:16540543